{
  "gene": "UniProtKB:Q8NDX9",
  "term_label": "external side of plasma membrane",
  "term_id": "GO:0009897",
  "gene_symbol": "LY6G5B",
  "gene_name": "Lymphocyte antigen 6 complex locus protein G5b"
}